forebrain neuroblast differentiation [GO:0021863] (biological process) References: PMID:16226447 Sources: GOC:cls, GOC:dgh, GOC:dph, GOC:jid, GO_REF:0000021 Also known as: abventricular progenitor cell differentiation, intermediate progenitor cell differentiation, non-surface dividing progenitor cell differentiation Definition: The process in which neuroepithelial cells in the neural tube acquire specialized structural and/or functional features of basal progenitor cells, neuroblasts that lose their contacts with the ventricular surface. Differentiation includes the processes involved in commitment of a cell to a specific fate. Relationships: is a type of neuroblast differentiation [GO:0014016]; is part of forebrain generation of neurons [GO:0021872]